{
  "term_label": "Unknown molecular function",
  "gene_symbol": "CYRIA",
  "gene": "UniProtKB:Q9H0Q0",
  "gene_name": "CYFIP-related Rac1 interactor A",
  "term_id": "UNKNOWN:0001"
}